{
  "gene_name": "Coiled-coil domain-containing protein 167",
  "term_label": "Unknown cellular component",
  "gene": "UniProtKB:Q9P0B6",
  "gene_symbol": "CCDC167",
  "term_id": "UNKNOWN:0003"
}